{
  "term_id": "GO:0003009",
  "gene": "UniProtKB:P45378",
  "term_label": "skeletal muscle contraction",
  "gene_symbol": "TNNT3",
  "gene_name": "Troponin T, fast skeletal muscle"
}